{
  "gene_name": "Ammonium transporter Rh type A",
  "gene_symbol": "RHAG",
  "gene": "UniProtKB:Q02094",
  "term_id": "GO:0097272",
  "term_label": "ammonium homeostasis"
}